{
  "gene_name": "5-hydroxytryptamine receptor 6",
  "term_label": "G protein-coupled receptor signaling pathway, coupled to cyclic nucleotide second messenger",
  "gene": "UniProtKB:P50406",
  "gene_symbol": "HTR6",
  "term_id": "GO:0007187"
}